regulation of canonical Wnt signaling pathway [GO:0060828] (biological process) Relationships: is_a regulation of Wnt signaling pathway [GO:0030111]; regulates canonical Wnt signaling pathway [GO:0060070] Definition: Any process that modulates the rate, frequency, or extent of the Wnt signaling pathway through beta-catenin, the series of molecular signals initiated by binding of a Wnt protein to a frizzled family receptor on the surface of the target cell, followed by propagation of the signal via beta-catenin, and ending with a change in transcription of target genes. Sources: GOC:dph, GOC:sdb_2009, GOC:tb Subtypes: negative regulation of canonical Wnt signaling pathway [GO:0090090], positive regulation of canonical Wnt signaling pathway [GO:0090263] Also known as: regulation of Wnt receptor signaling pathway through beta-catenin, regulation of canonical Wnt receptor signaling pathway, regulation of canonical Wnt receptor signalling pathway, regulation of canonical Wnt-activated signaling pathway, catenin import into nucleus, regulation of catenin import into nucleus, regulation of catenin protein nuclear translocation